{
  "gene": "UniProtKB:O76062",
  "term_label": "cholesterol biosynthetic process",
  "term_id": "GO:0006695",
  "gene_symbol": "TM7SF2",
  "gene_name": "Delta(14)-sterol reductase TM7SF2"
}